{
  "gene": "UniProtKB:Q9BXR5",
  "gene_name": "Toll-like receptor 10",
  "term_id": "GO:0002224",
  "gene_symbol": "TLR10",
  "term_label": "toll-like receptor signaling pathway"
}